{
  "term_id": "UNKNOWN:0001",
  "gene_name": "Cyclin N-terminal domain-containing protein 1",
  "term_label": "Unknown molecular function",
  "gene_symbol": "CNTD1",
  "gene": "UniProtKB:Q8N815"
}